{
  "term_id": "GO:0005802",
  "term_label": "trans-Golgi network",
  "gene_symbol": "AP4M1",
  "gene_name": "AP-4 complex subunit mu-1",
  "gene": "UniProtKB:O00189"
}